serine-type endopeptidase activity [GO:0004252] (molecular function) Also known as: blood coagulation factor activity, serine elastase activity Regulation: negatively regulated by serine-type endopeptidase inhibitor activity [GO:0004867]; regulated by regulation of serine-type endopeptidase activity [GO:1900003]; negatively regulated by negative regulation of serine-type endopeptidase activity [GO:1900004]; positively regulated by positive regulation of serine-type endopeptidase activity [GO:1900005] Relationships: is a type of endopeptidase activity [GO:0004175]; is a type of serine-type peptidase activity [GO:0008236] Sources: GOC:mah, https://www.ebi.ac.uk/merops/about/glossary.shtml#CATTYPE Definition: Catalysis of the hydrolysis of internal, alpha-peptide bonds in a polypeptide chain by a catalytic mechanism that involves a catalytic triad consisting of a serine nucleophile that is activated by a proton relay involving an acidic residue (e.g. aspartate or glutamate) and a basic residue (usually histidine).